{
  "term_label": "nucleus",
  "gene_name": "Interferon regulatory factor 1",
  "gene_symbol": "IRF1",
  "gene": "UniProtKB:P10914",
  "term_id": "GO:0005634"
}